{
  "term_id": "GO:0006357",
  "gene_name": "Interferon regulatory factor 9",
  "gene_symbol": "IRF9",
  "term_label": "regulation of transcription by RNA polymerase II",
  "gene": "UniProtKB:Q00978"
}